{
  "term_label": "double-stranded DNA binding",
  "gene_symbol": "GTF2H4",
  "term_id": "GO:0003690",
  "gene_name": "General transcription factor IIH subunit 4",
  "gene": "UniProtKB:Q92759"
}